{
  "term_label": "phosphatidylinositol transfer activity",
  "gene_name": "Membrane-associated phosphatidylinositol transfer protein 2",
  "gene": "UniProtKB:Q9BZ72",
  "term_id": "GO:0008526",
  "gene_symbol": "PITPNM2"
}